{
  "gene_symbol": "GSK3B",
  "term_id": "GO:0098978",
  "gene_name": "Glycogen synthase kinase-3 beta",
  "term_label": "glutamatergic synapse",
  "gene": "UniProtKB:P49841"
}